camera-type eye photoreceptor cell fate commitment [GO:0060220] (BP) Sources: GOC:dph Relationships: is a type of eye photoreceptor cell fate commitment [GO:0042706]; is part of camera-type eye photoreceptor cell differentiation [GO:0060219] Subtypes: retinal cone cell fate commitment [GO:0046551], retinal rod cell fate commitment [GO:0060223] Definition: The process in which the developmental fate of a cell becomes restricted such that it will develop into a photoreceptor cell in a camera-type eye.